{
  "gene_symbol": "FGF22",
  "gene": "UniProtKB:Q9HCT0",
  "gene_name": "Fibroblast growth factor 22",
  "term_label": "growth factor activity",
  "term_id": "GO:0008083"
}